4-hydroxyphenylacetaldehyde oxime monooxygenase activity [GO:0050592] (molecular function) Relationships: is a type of oxidoreductase activity, acting on paired donors, with incorporation or reduction of molecular oxygen, NAD(P)H as one donor, and incorporation of one atom of oxygen [GO:0016709] Sources: EC:1.14.14.37, RHEA:18401 Also known as: CYP71E1 activity, cytochrome P450-II-dependent monooxygenase activity, (Z)-4-hydroxyphenylacetaldehyde oxime,NADPH:oxygen oxidoreductase activity, 4-hydroxybenzeneacetaldehyde oxime monooxygenase activity, 4-hydroxyphenylacetaldehyde oxime,NADPH:oxygen oxidoreductase activity, NADPH-cytochrome P450 reductase (CYP71E1), cytochrome P450II-dependent monooxygenase activity Definition: Catalysis of the reaction: (Z)-(4-hydroxyphenyl)acetaldehyde oxime + H+ + NADPH + O2 = (S)-4-hydroxymandelonitrile + 2 H2O + NADP+.